{
  "gene_name": "Oxysterol-binding protein-related protein 1",
  "gene_symbol": "OSBPL1A",
  "term_id": "UNKNOWN:0002",
  "term_label": "Unknown biological process",
  "gene": "UniProtKB:Q9BXW6"
}